{
  "gene_name": "Adhesion G protein-coupled receptor E3",
  "term_label": "G protein-coupled receptor activity",
  "gene": "UniProtKB:Q9BY15",
  "term_id": "GO:0004930",
  "gene_symbol": "ADGRE3"
}